{
  "term_label": "Unknown cellular component",
  "gene_symbol": "UMAD1",
  "gene_name": "UBAP1-MVB12-associated (UMA)-domain containing protein 1",
  "term_id": "UNKNOWN:0003",
  "gene": "UniProtKB:C9J7I0"
}